{
  "term_id": "GO:0016324",
  "gene": "UniProtKB:P08183",
  "gene_name": "ATP-dependent translocase ABCB1",
  "gene_symbol": "ABCB1",
  "term_label": "apical plasma membrane"
}